pre-mRNA intronic pyrimidine-rich binding [GO:0097158] (molecular function) References: PMID:16260624, PMID:16777844 Sources: GOC:ans Relationships: is a type of pre-mRNA intronic binding [GO:0097157] Also known as: pre-messenger RNA intronic pyrimidine-rich binding Definition: Binding to a pyrimidine-rich (CU-rich) intronic sequence of a pre-messenger RNA (pre-mRNA).